{
  "term_label": "signal transduction",
  "gene_symbol": "FCAMR",
  "gene_name": "High affinity immunoglobulin alpha and immunoglobulin mu Fc receptor",
  "gene": "UniProtKB:Q8WWV6",
  "term_id": "GO:0007165"
}